nectar secretion [GO:0071836] (biological process) Also known as: nectar production Relationships: is_a secretion [GO:0046903] Definition: The controlled release of a nectar by a cell or a tissue. Nectar is a fluid secreted by many angiosperms to promote pollination by providing a reward to pollinators. Nectar may also deter certain organisms from visiting or play other biological roles. Nectar is a complex solution that may include the following types of compounds: sugars, amino acids, organic acids, alkaloids, flavonoids, glycosides, vitamins, phenolics, metal ions, oils, free fatty acids, and proteins. References: PMID:19861655 Sources: GOC:kad